glutaryl-CoA dehydrogenase activity [GO:0004361] (molecular function) Relationships: is a type of acyl-CoA dehydrogenase activity [GO:0003995] Also known as: glutaryl coenzyme A dehydrogenase activity Sources: RHEA:13389 Definition: Catalysis of the reaction: glutaryl-CoA + 2 H+ + oxidized [electron-transfer flavoprotein] = (2E)-butenoyl-CoA + CO2 + reduced [electron-transfer flavoprotein].